{
  "term_id": "GO:0007602",
  "term_label": "phototransduction",
  "gene": "UniProtKB:Q9UHM6",
  "gene_symbol": "OPN4",
  "gene_name": "Melanopsin"
}